{
  "gene": "UniProtKB:A6NMB9",
  "gene_symbol": "FIGNL2",
  "term_id": "GO:0016887",
  "term_label": "ATP hydrolysis activity",
  "gene_name": "Fidgetin-like protein 2"
}